{
  "gene_name": "Mediator of RNA polymerase II transcription subunit 1",
  "gene": "UniProtKB:Q15648",
  "gene_symbol": "MED1",
  "term_id": "GO:0016592",
  "term_label": "mediator complex"
}